{
  "gene": "UniProtKB:Q96RT8",
  "term_label": "gamma-tubulin complex",
  "term_id": "GO:0000930",
  "gene_name": "Gamma-tubulin complex component 5",
  "gene_symbol": "TUBGCP5"
}